{
  "gene": "UniProtKB:Q96G74",
  "gene_symbol": "OTUD5",
  "term_label": "K63-linked deubiquitinase activity",
  "gene_name": "OTU domain-containing protein 5",
  "term_id": "GO:0061578"
}